hepatocyte apoptotic process [GO:0097284] (biological process) Relationships: is a type of GO:1904019 Regulation: regulated by regulation of hepatocyte apoptotic process [GO:1903943]; negatively regulated by negative regulation of hepatocyte apoptotic process [GO:1903944]; positively regulated by positive regulation of hepatocyte apoptotic process [GO:1903945] References: PMID:15856020 Sources: CL:0000182, GOC:jc, GOC:mtg_apoptosis Definition: Any apoptotic process in a hepatocyte, the main structural component of the liver. Also known as: hepatocyte apoptosis